{
  "gene_name": "DNA-directed RNA polymerase II subunit RPB11-b2",
  "gene": "UniProtKB:Q9H1A7",
  "gene_symbol": "POLR2J3",
  "term_label": "DNA-directed RNA polymerase activity",
  "term_id": "GO:0003899"
}